{
  "term_label": "phospholipid binding",
  "gene": "UniProtKB:Q9Y6I3",
  "term_id": "GO:0005543",
  "gene_symbol": "EPN1",
  "gene_name": "Epsin-1"
}